disulfide oxidoreductase activity [GO:0015036] (molecular function) Subtypes: GO:0015035, GO:0015038, trypanothione-disulfide reductase (NADPH) activity [GO:0015042], GO:0016972, CoA-disulfide reductase (NADPH) activity [GO:0050451], selenodiglutathione-disulfide reductase (NADPH) activity [GO:0098622], GO:0141049 Sources: GOC:curators Relationships: is a type of oxidoreductase activity, acting on a sulfur group of donors [GO:0016667] Also known as: disulphide oxidoreductase activity Definition: Catalysis of the reaction: substrate with reduced sulfide groups = substrate with oxidized disulfide bonds.